{
  "term_id": "GO:0007165",
  "gene": "UniProtKB:Q86YV6",
  "gene_symbol": "MYLK4",
  "term_label": "signal transduction",
  "gene_name": "Myosin light chain kinase family member 4"
}